{
  "term_id": "GO:0019898",
  "term_label": "extrinsic component of membrane",
  "gene": "UniProtKB:Q96PX9",
  "gene_symbol": "PLEKHG4B",
  "gene_name": "Pleckstrin homology domain-containing family G member 4B"
}